{
  "gene": "UniProtKB:A2AJT9",
  "term_label": "positive regulation of transcription by RNA polymerase II",
  "gene_name": "BCLAF1 and THRAP3 family member 3",
  "term_id": "GO:0045944",
  "gene_symbol": "BCLAF3"
}